taurine binding [GO:0030977] (molecular function) Relationships: is a type of alkanesulfonate binding [GO:0043210] Definition: Binding to taurine. Sources: GOC:mlg